{
  "gene": "UniProtKB:Q9Y2X9",
  "term_id": "GO:0000978",
  "term_label": "RNA polymerase II cis-regulatory region sequence-specific DNA binding",
  "gene_name": "Zinc finger protein 281",
  "gene_symbol": "ZNF281"
}